{
  "gene_name": "MHC class I polypeptide-related sequence A",
  "term_label": "extracellular space",
  "gene_symbol": "MICA",
  "term_id": "GO:0005615",
  "gene": "UniProtKB:Q29983"
}